{
  "gene_name": "Olfactory receptor 5H15",
  "gene": "UniProtKB:A6NDH6",
  "gene_symbol": "OR5H15",
  "term_id": "UNKNOWN:0003",
  "term_label": "Unknown cellular component"
}